{
  "gene": "UniProtKB:Q9P265",
  "gene_name": "Disco-interacting protein 2 homolog B",
  "term_label": "Unknown biological process",
  "term_id": "UNKNOWN:0002",
  "gene_symbol": "DIP2B"
}